detection of jasmonic acid stimulus [GO:0009754] (biological process) Sources: GOC:sm Definition: The series of events in which a jasmonic acid stimulus is received by a cell and converted into a molecular signal. Series of events required for a jasmonic acid stimulus to be detected and converted to a signal molecule. Relationships: is a type of detection of chemical stimulus [GO:0009593]; is a type of response to jasmonic acid [GO:0009753] Also known as: perception of jasmonic acid stimulus